{
  "gene_symbol": "HYPK",
  "term_id": "UNKNOWN:0001",
  "gene_name": "Huntingtin-interacting protein K",
  "term_label": "Unknown molecular function",
  "gene": "UniProtKB:Q9NX55"
}